positive regulation of fusion of virus membrane with host plasma membrane [GO:1903915] (biological process) References: PMID:23575248 Sources: GOC:TermGenie, GOC:als, GO_REF:0000058 Relationships: is a type of GO:0046598; is a type of GO:0051130; is a type of GO:1903913; positively regulates fusion of virus membrane with host plasma membrane [GO:0019064] Definition: Any process that activates or increases the frequency, rate or extent of fusion of virus membrane with host plasma membrane. Also known as: positive regulation of viral envelope fusion with host cell membrane, positive regulation of viral envelope fusion with host membrane, positive regulation of viral envelope fusion with host plasma membrane, positive regulation of viral penetration via membrane fusion, up regulation of fusion of virus membrane with host plasma membrane, up regulation of viral envelope fusion with host cell membrane, up regulation of viral envelope fusion with host membrane, up regulation of viral envelope fusion with host plasma membrane, up regulation of viral penetration via membrane fusion, up-regulation of fusion of virus membrane with host plasma membrane, up-regulation of viral envelope fusion with host cell membrane, up-regulation of viral envelope fusion with host membrane, up-regulation of viral envelope fusion with host plasma membrane, up-regulation of viral penetration via membrane fusion, upregulation of fusion of virus membrane with host plasma membrane, upregulation of viral envelope fusion with host cell membrane, upregulation of viral envelope fusion with host membrane, upregulation of viral envelope fusion with host plasma membrane, upregulation of viral penetration via membrane fusion, activation of fusion of virus membrane with host plasma membrane, activation of viral envelope fusion with host cell membrane, activation of viral envelope fusion with host membrane, activation of viral envelope fusion with host plasma membrane, activation of viral penetration via membrane fusion, activation of viral entry into host cell via membrane fusion with the plasma membrane, activation of viral-cell fusion molecule activity, positive regulation of viral entry into host cell via membrane fusion with the plasma membrane, positive regulation of viral-cell fusion molecule activity, up regulation of viral entry into host cell via membrane fusion with the plasma membrane, up regulation of viral-cell fusion molecule activity, up-regulation of viral entry into host cell via membrane fusion with the plasma membrane, up-regulation of viral-cell fusion molecule activity, upregulation of viral entry into host cell via membrane fusion with the plasma membrane, upregulation of viral-cell fusion molecule activity